{
  "gene_symbol": "ZNF200",
  "gene": "UniProtKB:P98182",
  "term_label": "Unknown biological process",
  "term_id": "UNKNOWN:0002",
  "gene_name": "Zinc finger protein 200"
}